{
  "gene_name": "Peroxisome biogenesis factor 2",
  "gene": "UniProtKB:P28328",
  "gene_symbol": "PEX2",
  "term_id": "GO:0000038",
  "term_label": "very long-chain fatty acid metabolic process"
}